{
  "gene_symbol": "CRH",
  "term_label": "extracellular space",
  "term_id": "GO:0005615",
  "gene_name": "Corticoliberin",
  "gene": "UniProtKB:P06850"
}